SAGA complex assembly [GO:0036285] (biological process) Also known as: SAGA complex formation Relationships: is a type of GO:0065003 Definition: The aggregation, arrangement and bonding together of a set of components to form a SAGA complex, a SAGA-type histone acetyltransferase complex that contains Spt8 (in budding yeast) or a homolog thereof. References: PMID:10637607, PMID:22456315 Sources: GOC:mah